positive regulation of metanephric ureteric bud development [GO:2001076] (biological process) Sources: GOC:obol Definition: Any process that activates or increases the frequency, rate or extent of metanephric ureteric bud development. Relationships: is_a GO:0051094; is a type of regulation of metanephric ureteric bud development [GO:2001074]; positively regulates GO:0035502